{
  "gene_symbol": "MAP3K8",
  "term_label": "MAPK cascade",
  "term_id": "GO:0000165",
  "gene_name": "Mitogen-activated protein kinase kinase kinase 8",
  "gene": "UniProtKB:P41279"
}